{
  "term_label": "zinc ion transport",
  "gene": "UniProtKB:Q6PML9",
  "term_id": "GO:0006829",
  "gene_symbol": "SLC30A9",
  "gene_name": "Proton-coupled zinc antiporter SLC30A9, mitochondrial"
}